{
  "gene_symbol": "OR5AU1",
  "gene_name": "Olfactory receptor 5AU1",
  "gene": "UniProtKB:Q8NGC0",
  "term_id": "UNKNOWN:0002",
  "term_label": "Unknown biological process"
}